{
  "gene": "UniProtKB:O95342",
  "gene_name": "Bile salt export pump",
  "term_label": "apical plasma membrane",
  "term_id": "GO:0016324",
  "gene_symbol": "ABCB11"
}